{
  "term_label": "sulfotransferase activity",
  "gene_symbol": "CHST14",
  "gene": "UniProtKB:Q8NCH0",
  "term_id": "GO:0008146",
  "gene_name": "Carbohydrate sulfotransferase 14"
}